{
  "term_label": "receptor recycling",
  "gene": "UniProtKB:Q8N4B1",
  "gene_symbol": "PHETA1",
  "gene_name": "Sesquipedalian-1",
  "term_id": "GO:0001881"
}